ethanolamine degradation polyhedral organelle [GO:0031471] (cellular component) Definition: An organelle found in bacteria consisting of a proteinaceous coat containing enzymes for the degradation of ethanolamine whose purpose is the protection of the rest of the cell from the toxic acetaldehyde product of the enzyme ethanolamine ammonia lyase. References: PMID:11844753 Sources: GOC:js Also known as: ethanolamine metabolosome Relationships: is a type of bacterial microcompartment [GO:0031469]